{
  "gene_name": "Homeobox protein Meis2",
  "gene": "UniProtKB:O14770",
  "term_id": "GO:0001228",
  "term_label": "DNA-binding transcription activator activity, RNA polymerase II-specific",
  "gene_symbol": "MEIS2"
}